{
  "term_label": "helper T cell enhancement of adaptive immune response",
  "term_id": "GO:0035397",
  "gene_name": "T-cell surface glycoprotein CD4",
  "gene_symbol": "CD4",
  "gene": "UniProtKB:P01730"
}